{
  "gene": "UniProtKB:Q13838",
  "gene_symbol": "DDX39B",
  "term_label": "mRNA export from nucleus",
  "gene_name": "Spliceosome RNA helicase DDX39B",
  "term_id": "GO:0006406"
}